{
  "gene": "UniProtKB:P22674",
  "term_id": "GO:0005737",
  "term_label": "cytoplasm",
  "gene_name": "Cyclin-O",
  "gene_symbol": "CCNO"
}